5-valerolactone hydrolase activity [GO:0055042] (molecular function) Definition: Catalysis of the reaction: 5-valerolactone + H2O = 5-hydroxyvalerate. Sources: GOC:jid, GOC:mlg Relationships: is a type of GO:0046573